{
  "gene": "UniProtKB:P11279",
  "term_label": "late endosome membrane",
  "gene_name": "Lysosome-associated membrane glycoprotein 1",
  "gene_symbol": "LAMP1",
  "term_id": "GO:0031902"
}